{
  "gene_name": "Olfactory receptor 10A4",
  "term_id": "GO:0050911",
  "gene": "UniProtKB:Q9H209",
  "gene_symbol": "OR10A4",
  "term_label": "detection of chemical stimulus involved in sensory perception of smell"
}